{
  "gene_symbol": "SLAMF1",
  "term_label": "immune response",
  "gene_name": "Signaling lymphocytic activation molecule",
  "gene": "UniProtKB:Q13291",
  "term_id": "GO:0006955"
}